{
  "term_id": "UNKNOWN:0003",
  "gene_symbol": "CASC2",
  "gene": "UniProtKB:Q6XLA1",
  "gene_name": "Protein CASC2, isoform 3",
  "term_label": "Unknown cellular component"
}